RNA polymerase I transcription regulatory region sequence-specific DNA binding [GO:0001163] (molecular function) Sources: GOC:txnOH Also known as: RNA polymerase I regulatory region DNA binding Definition: Binding to a specific sequence of DNA that is part of a regulatory region that controls the transcription of a gene or cistron by RNA polymerase I. Subtypes: RNA polymerase I core promoter sequence-specific DNA binding [GO:0001164], GO:0001165 Relationships: is a type of transcription cis-regulatory region binding [GO:0000976]